trans-2,3-dihydro-3-hydroxy-anthranilate isomerase activity [GO:0102943] (molecular function) Definition: Catalysis of the reaction: (2S,3S)-2,3-dihydro-3-hydroxyanthranilic acid = (1R,6S)-6-ammonio-5-oxocyclohex-2-ene-1-carboxylate. Sources: GOC:pz, RHEA:28182 Relationships: is a type of intramolecular oxidoreductase activity, transposing C=C bonds [GO:0016863]